{
  "gene_symbol": "RAB33A",
  "term_id": "GO:0005525",
  "term_label": "GTP binding",
  "gene_name": "Ras-related protein Rab-33A",
  "gene": "UniProtKB:Q14088"
}